{
  "gene_symbol": "KRT19",
  "gene": "UniProtKB:P08727",
  "gene_name": "Keratin, type I cytoskeletal 19",
  "term_id": "GO:0005856",
  "term_label": "cytoskeleton"
}